microlipophagy [GO:0140504] (biological process) References: PMID:25070953, PMID:28394250, PMID:28838958, PMID:29293450, PMID:29601311 Definition: Degradation of a lipid droplet by microautophagy. Regulation: regulated by regulation of microlipophagy [GO:0140505] Also known as: lipid droplet autophagy Relationships: is a type of microautophagy [GO:0016237]